{
  "term_id": "GO:0051603",
  "gene_symbol": "IDE",
  "gene_name": "Insulin-degrading enzyme",
  "term_label": "proteolysis involved in protein catabolic process",
  "gene": "UniProtKB:P14735"
}